{
  "term_label": "Unknown cellular component",
  "gene_name": "B melanoma antigen 5",
  "gene_symbol": "BAGE5",
  "term_id": "UNKNOWN:0003",
  "gene": "UniProtKB:Q86Y27"
}